zygosporangium development [GO:0075271] (biological process) Definition: The process in which a fruiting body called zygosporangium is formed. A zygosporangium is a thick-walled structure in which spores are produced, and is characteristic of the Zygomycetes. Regulation: regulated by regulation of zygosporangium development [GO:0075272]; positively regulated by GO:0075273; negatively regulated by negative regulation of zygosporangium development [GO:0075274] Sources: GOC:pamgo_curators Relationships: is a type of spore-bearing structure development [GO:0075259]